shelterin complex [GO:0070187] (cellular component) References: PMID:18828880 Sources: GOC:expert_mf, GOC:mah, GOC:vw Relationships: is a type of GO:0000783 Definition: A nuclear telomere cap complex that is formed by the association of telomeric ssDNA- and dsDNA-binding proteins with telomeric DNA, and is involved in telomere protection and recruitment of telomerase. The complex is known to contain TERF1, TERF2, POT1, RAP1, TINF2 and ACD in mammalian cells, and Pot1, Tpz1, Rap1, Rif1, Rif2 and Taz1 in Saccharomyces. Taz1 and Rap1 (or their mammalian equivalents) form a dsDNA-binding subcomplex, Pot1 and Tpz1 form an ssDNA-binding subcomplex, and the two subcomplexes are bridged by Poz1, which acts as an effector molecule along with Ccq1. Also known as: Pot1 complex, Pot1-Tpz1 complex, telosome